{
  "gene": "UniProtKB:Q9BZL1",
  "term_id": "GO:0005737",
  "gene_symbol": "UBL5",
  "gene_name": "Ubiquitin-like protein 5",
  "term_label": "cytoplasm"
}